catenin complex [GO:0016342] (cellular component) Relationships: is a type of plasma membrane protein complex [GO:0098797]; is part of extrinsic component of plasma membrane [GO:0019897] Definition: Complex of peripheral cytoplasmic proteins (alpha-, beta- and gamma-catenin) that interact with the cytoplasmic region of uvomorulin/E-cadherin to connect it to the actin cytoskeleton. Sources: ISBN:0198599323